{
  "gene_symbol": "SSTR1",
  "term_id": "GO:0043005",
  "gene": "UniProtKB:P30872",
  "term_label": "neuron projection",
  "gene_name": "Somatostatin receptor type 1"
}